{
  "term_label": "glucuronosyltransferase activity",
  "term_id": "GO:0015020",
  "gene": "UniProtKB:Q16394",
  "gene_name": "Exostosin-1",
  "gene_symbol": "EXT1"
}